{
  "gene_name": "Androglobin",
  "term_id": "GO:0097227",
  "gene_symbol": "ADGB",
  "term_label": "sperm annulus",
  "gene": "UniProtKB:Q8N7X0"
}